{
  "gene": "UniProtKB:Q9UPW6",
  "term_label": "Unknown cellular component",
  "gene_symbol": "SATB2",
  "term_id": "UNKNOWN:0003",
  "gene_name": "DNA-binding protein SATB2"
}